{
  "term_label": "Unknown cellular component",
  "gene": "UniProtKB:A1L453",
  "gene_name": "Serine protease 38",
  "gene_symbol": "PRSS38",
  "term_id": "UNKNOWN:0003"
}